{
  "gene_symbol": "OR2G6",
  "gene": "UniProtKB:Q5TZ20",
  "term_label": "plasma membrane",
  "term_id": "GO:0005886",
  "gene_name": "Olfactory receptor 2G6"
}